{
  "gene_name": "C-X-C chemokine receptor type 4",
  "gene": "UniProtKB:P61073",
  "term_label": "brain development",
  "term_id": "GO:0007420",
  "gene_symbol": "CXCR4"
}